{
  "gene": "UniProtKB:P0DN82",
  "term_label": "olfactory receptor activity",
  "gene_symbol": "OR12D1",
  "term_id": "GO:0004984",
  "gene_name": "Olfactory receptor 12D1"
}